{
  "term_label": "glutathione disulfide oxidoreductase activity",
  "term_id": "GO:0015038",
  "gene": "UniProtKB:P35754",
  "gene_symbol": "GLRX",
  "gene_name": "Glutaredoxin-1"
}